{
  "term_id": "GO:0007219",
  "gene": "UniProtKB:O14672",
  "term_label": "Notch signaling pathway",
  "gene_symbol": "ADAM10",
  "gene_name": "Disintegrin and metalloproteinase domain-containing protein 10"
}